{
  "gene_name": "TNF receptor-associated factor 4",
  "term_id": "GO:0007166",
  "term_label": "cell surface receptor signaling pathway",
  "gene": "UniProtKB:Q9BUZ4",
  "gene_symbol": "TRAF4"
}